{
  "gene": "UniProtKB:Q9H6D7",
  "term_id": "GO:0070652",
  "gene_symbol": "HAUS4",
  "gene_name": "HAUS augmin-like complex subunit 4",
  "term_label": "HAUS complex"
}